{
  "gene": "UniProtKB:Q9C010",
  "gene_symbol": "PKIB",
  "gene_name": "cAMP-dependent protein kinase inhibitor beta",
  "term_label": "nucleus",
  "term_id": "GO:0005634"
}